{
  "term_id": "GO:0043410",
  "gene_symbol": "FLT1",
  "gene_name": "Vascular endothelial growth factor receptor 1",
  "term_label": "positive regulation of MAPK cascade",
  "gene": "UniProtKB:P17948"
}